{
  "term_label": "Unknown biological process",
  "gene_symbol": "MRPL46",
  "term_id": "UNKNOWN:0002",
  "gene": "UniProtKB:Q9H2W6",
  "gene_name": "Large ribosomal subunit protein mL46"
}